P2 peroxisome [GO:0019820] (cellular component) Also known as: peroxisome vesicle References: PMID:10629216 Definition: A subform of peroxisome that corresponds to an intermediate in a peroxisome assembly pathway, which operates by conversion of peroxisomal subforms in the direction P1, P2 -> P3 -> P4 -> P5 -> P6. P2 peroxisomes are distinguished from the other subforms on the bases of buoyant density and protein content; they are the least dense of the subforms observed. Relationships: is a type of peroxisome [GO:0005777] Note: Note that this peroxisome assembly pathway is described in the yeast Yarrowia lipolytica. See also the cellular component terms 'P1 peroxisome ; GO:0019819', 'P3 peroxisome ; GO:0019821', 'P4 peroxisome ; GO:0019822', 'P5 peroxisome ; GO:0019823', and 'P6 peroxisome ; GO:0019824'.